{
  "term_id": "GO:0001228",
  "gene": "UniProtKB:Q8N554",
  "term_label": "DNA-binding transcription activator activity, RNA polymerase II-specific",
  "gene_symbol": "ZNF276",
  "gene_name": "Zinc finger protein 276"
}